positive regulation of leukocyte degranulation [GO:0043302] (biological process) Definition: Any process that activates or increases the frequency, rate or extent of leukocyte degranulation. Sources: GOC:add, ISBN:0781735149 Relationships: is a type of GO:0002699; is a type of regulation of leukocyte degranulation [GO:0043300]; is a type of GO:1903307; positively regulates leukocyte degranulation [GO:0043299] Also known as: positive regulation of immune cell degranulation, positive regulation of leucocyte degranulation, up regulation of leukocyte degranulation, up-regulation of leukocyte degranulation, upregulation of leukocyte degranulation, activation of leukocyte degranulation, stimulation of leukocyte degranulation Subtypes: positive regulation of mast cell degranulation [GO:0043306], GO:0043311, GO:0043315, positive regulation of cytotoxic T cell degranulation [GO:0043319], positive regulation of natural killer cell degranulation [GO:0043323], positive regulation of basophil degranulation [GO:1903583]